geraniol catabolic process [GO:1903447] (biological process) Relationships: is a type of polyprenol catabolic process [GO:0016095]; is a type of GO:0016100; is_a GO:0034310; is a type of olefinic compound catabolic process [GO:0120256] Definition: The chemical reactions and pathways resulting in the breakdown of geraniol. References: PMID:23200656 Sources: GOC:TermGenie, GOC:di, GO_REF:0000068 Also known as: geraniol breakdown, geraniol catabolism, geraniol degradation